{
  "term_id": "GO:0140359",
  "gene_symbol": "ABCC4",
  "gene": "UniProtKB:O15439",
  "gene_name": "ATP-binding cassette sub-family C member 4",
  "term_label": "ABC-type transporter activity"
}